{
  "term_id": "GO:0005484",
  "gene_name": "Syntaxin-17",
  "term_label": "SNAP receptor activity",
  "gene": "UniProtKB:P56962",
  "gene_symbol": "STX17"
}